{
  "term_id": "GO:0005814",
  "gene_name": "Protein NEDD1",
  "term_label": "centriole",
  "gene": "UniProtKB:Q8NHV4",
  "gene_symbol": "NEDD1"
}